{
  "gene_name": "Ephrin type-A receptor 5",
  "gene_symbol": "EPHA5",
  "gene": "UniProtKB:P54756",
  "term_id": "GO:0007411",
  "term_label": "axon guidance"
}